{
  "term_label": "cell chemotaxis",
  "gene_name": "C-C motif chemokine 15",
  "term_id": "GO:0060326",
  "gene_symbol": "CCL15",
  "gene": "UniProtKB:Q16663"
}